{
  "gene_symbol": "SNX2",
  "gene": "UniProtKB:O60749",
  "term_id": "GO:0035091",
  "term_label": "phosphatidylinositol binding",
  "gene_name": "Sorting nexin-2"
}